UDP-glucosyltransferase activity [GO:0035251] (molecular function) Relationships: is a type of UDP-glycosyltransferase activity [GO:0008194]; is a type of glucosyltransferase activity [GO:0046527] References: PMID:19858195 Subtypes: GO:0003825, 1,3-beta-D-glucan synthase activity [GO:0003843], UDP-glucose:glycoprotein glucosyltransferase activity [GO:0003980], alpha-1,4-glucan glucosyltransferase (UDP-glucose donor) activity [GO:0004373], dolichyl-phosphate beta-glucosyltransferase activity [GO:0004581], ceramide glucosyltransferase activity [GO:0008120], glycogenin glucosyltransferase activity [GO:0008466], GO:0008919, abscisic acid glucosyltransferase activity [GO:0010294], GO:0016157, cellulose synthase (UDP-forming) activity [GO:0016760], GO:0016906, sucrose-phosphate synthase activity [GO:0046524], o-dihydroxycoumarin 7-O-glucosyltransferase activity [GO:0047208], coniferyl-alcohol glucosyltransferase activity [GO:0047209], 2-coumarate O-beta-glucosyltransferase activity [GO:0047212], anthocyanidin 3-O-glucosyltransferase activity [GO:0047213], cyanidin-3-rhamnosylglucoside 5-O-glucosyltransferase activity [GO:0047214], indole-3-acetate beta-glucosyltransferase activity [GO:0047215], GO:0047218, GO:0047219, GO:0047228, GO:0047229, pyridoxine 5'-O-beta-D-glucosyltransferase activity [GO:0047231], GO:0047236, hydroxymandelonitrile glucosyltransferase activity [GO:0047239], hydroxyanthraquinone glucosyltransferase activity [GO:0047242], flavanone 7-O-beta-glucosyltransferase activity [GO:0047243], GO:0047245, GO:0047248, sarsapogenin 3-beta-glucosyltransferase activity [GO:0047249], GO:0047250, GO:0047251, 2,4-dihydroxy-7-methoxy-2H-1,4-benzoxazin-3(4H)-one 2-D-glucosyltransferase activity [GO:0047254], poly(glycerol-phosphate) alpha-glucosyltransferase activity [GO:0047265], poly(ribitol-phosphate) beta-glucosyltransferase activity [GO:0047266], GO:0047270, phosphopolyprenol glucosyltransferase activity [GO:0047272], alizarin 2-beta-glucosyltransferase activity [GO:0047644], GO:0047684, cyanohydrin beta-glucosyltransferase activity [GO:0047792], GO:0047807, flavone 7-O-beta-glucosyltransferase activity [GO:0047891], flavonol 3-O-glucosyltransferase activity [GO:0047893], gallate 1-beta-glucosyltransferase activity [GO:0047913], GO:0047928, isoflavone 7-O-glucosyltransferase activity [GO:0050004], isovitexin beta-glucosyltransferase activity [GO:0050010], nicotinate-N-glucosyltransferase activity [GO:0050139], phenol beta-glucosyltransferase activity [GO:0050171], salicyl-alcohol beta-D-glucosyltransferase activity [GO:0050274], GO:0050275, sinapate 1-glucosyltransferase activity [GO:0050284], vitexin beta-glucosyltransferase activity [GO:0050395], trans-zeatin O-beta-D-glucosyltransferase activity [GO:0050403], cinnamate beta-D-glucosyltransferase activity [GO:0050412], ecdysteroid UDP-glucosyltransferase activity [GO:0050488], cis-zeatin O-beta-D-glucosyltransferase activity [GO:0050502], hydroquinone glucosyltransferase activity [GO:0050505], GO:0050506, indoxyl-UDPG glucosyltransferase activity [GO:0050507], GO:0050644, limonoid glucosyltransferase activity [GO:0050645], indole-3-butyrate beta-glucosyltransferase activity [GO:0052638], GO:0052639, salicylic acid glucosyltransferase (glucoside-forming) activity [GO:0052640], benzoic acid glucosyltransferase activity [GO:0052641], UDP-glucose:4-aminobenzoate acylglucosyltransferase activity [GO:0080002], anthocyanin 5-O-glucosyltransferase activity [GO:0080018], quercetin 3-O-glucosyltransferase activity [GO:0080043], quercetin 7-O-glucosyltransferase activity [GO:0080044], quercetin 3'-O-glucosyltransferase activity [GO:0080045], GO:0080046, GO:0080062, GO:0090704, GO:0140561, O-fucosylpeptide 3-beta-glucosyltransferase activity [GO:0160265] Definition: Catalysis of the transfer of a glucosyl group from UDP-glucose to an acceptor molecule.